{
  "term_label": "Unknown molecular function",
  "term_id": "UNKNOWN:0001",
  "gene_name": "Centriolar and ciliogenesis-associated protein HYLS1",
  "gene": "UniProtKB:Q96M11",
  "gene_symbol": "HYLS1"
}